{
  "gene_symbol": "ADGRB1",
  "gene": "UniProtKB:O14514",
  "gene_name": "Adhesion G protein-coupled receptor B1",
  "term_id": "GO:0005886",
  "term_label": "plasma membrane"
}